{
  "gene_symbol": "YWHAZ",
  "term_id": "GO:0005737",
  "gene": "UniProtKB:P63104",
  "term_label": "cytoplasm",
  "gene_name": "14-3-3 protein zeta_delta"
}